{
  "term_label": "RNA polymerase II transcription regulatory region sequence-specific DNA binding",
  "term_id": "GO:0000977",
  "gene_name": "Homeobox protein ESX1",
  "gene_symbol": "ESX1",
  "gene": "UniProtKB:Q8N693"
}